{
  "term_label": "detection of chemical stimulus involved in sensory perception of smell",
  "gene_symbol": "OR2C3",
  "gene_name": "Olfactory receptor 2C3",
  "term_id": "GO:0050911",
  "gene": "UniProtKB:Q8N628"
}